{
  "gene_symbol": "BTLA",
  "term_label": "plasma membrane",
  "gene": "UniProtKB:Q7Z6A9",
  "gene_name": "B- and T-lymphocyte attenuator",
  "term_id": "GO:0005886"
}